{
  "gene_symbol": "PID1",
  "term_label": "Unknown molecular function",
  "gene": "UniProtKB:Q7Z2X4",
  "term_id": "UNKNOWN:0001",
  "gene_name": "PTB-containing, cubilin and LRP1-interacting protein"
}